{
  "gene_name": "Vacuolar protein sorting-associated protein 33B",
  "gene_symbol": "VPS33B",
  "term_label": "intracellular protein transport",
  "gene": "UniProtKB:Q9H267",
  "term_id": "GO:0006886"
}